{
  "term_label": "Golgi apparatus",
  "gene": "UniProtKB:Q14435",
  "term_id": "GO:0005794",
  "gene_name": "Polypeptide N-acetylgalactosaminyltransferase 3",
  "gene_symbol": "GALNT3"
}